{
  "gene_name": "Metallothionein-1A",
  "term_label": "intracellular zinc ion homeostasis",
  "term_id": "GO:0006882",
  "gene": "UniProtKB:P04731",
  "gene_symbol": "MT1A"
}